{
  "gene_symbol": "ADCY9",
  "term_id": "GO:0007189",
  "gene_name": "Adenylate cyclase type 9",
  "term_label": "adenylate cyclase-activating G protein-coupled receptor signaling pathway",
  "gene": "UniProtKB:O60503"
}